{
  "gene": "UniProtKB:P25311",
  "term_id": "UNKNOWN:0001",
  "gene_symbol": "AZGP1",
  "term_label": "Unknown molecular function",
  "gene_name": "Zinc-alpha-2-glycoprotein"
}